{
  "gene_name": "Peroxisomal membrane protein PMP34",
  "term_id": "UNKNOWN:0002",
  "term_label": "Unknown biological process",
  "gene_symbol": "SLC25A17",
  "gene": "UniProtKB:O43808"
}